{
  "gene": "UniProtKB:Q0VF49",
  "gene_name": "Uncharacterized protein KIAA2012",
  "term_id": "UNKNOWN:0001",
  "gene_symbol": "KIAA2012",
  "term_label": "Unknown molecular function"
}